detection of humidity stimulus involved in sensory perception [GO:0098512] (biological process) Subtypes: GO:0098514, detection of low humidity stimulus involved in sensory perception [GO:0098515] Relationships: is a type of detection of stimulus involved in sensory perception [GO:0050906]; is a type of detection of humidity [GO:0098513]; is part of sensory perception of humidity [GO:0098509] Definition: The series of events in which a humidity stimulus is received and converted into a molecular signal as part of the sensory perception of humidity. References: PMID:8650222 Sources: GOC:dos